{
  "gene": "UniProtKB:Q96PQ6",
  "gene_name": "Zinc finger protein 317",
  "term_id": "GO:0000981",
  "gene_symbol": "ZNF317",
  "term_label": "DNA-binding transcription factor activity, RNA polymerase II-specific"
}